{
  "gene_name": "Polyubiquitin-B",
  "term_label": "protein tag activity",
  "gene_symbol": "UBB",
  "term_id": "GO:0031386",
  "gene": "UniProtKB:P0CG47"
}